{
  "term_id": "GO:0048255",
  "gene_name": "Terminal nucleotidyltransferase 5D",
  "term_label": "mRNA stabilization",
  "gene": "UniProtKB:Q8NEK8",
  "gene_symbol": "TENT5D"
}